{
  "term_id": "GO:0005634",
  "gene_name": "DnaJ homolog subfamily C member 8",
  "gene": "UniProtKB:O75937",
  "term_label": "nucleus",
  "gene_symbol": "DNAJC8"
}